{
  "gene_symbol": "GDF5",
  "term_id": "GO:0005615",
  "gene": "UniProtKB:P43026",
  "term_label": "extracellular space",
  "gene_name": "Growth_differentiation factor 5"
}